{
  "gene_name": "Nuclear factor erythroid 2-related factor 2",
  "gene": "UniProtKB:Q16236",
  "gene_symbol": "NFE2L2",
  "term_label": "RNA polymerase II cis-regulatory region sequence-specific DNA binding",
  "term_id": "GO:0000978"
}